{
  "gene": "UniProtKB:Q9Y6U3",
  "term_label": "cell projection assembly",
  "gene_name": "Scinderin",
  "gene_symbol": "SCIN",
  "term_id": "GO:0030031"
}